{
  "gene_name": "PiggyBac transposable element-derived protein 4",
  "term_id": "UNKNOWN:0001",
  "term_label": "Unknown molecular function",
  "gene_symbol": "PGBD4",
  "gene": "UniProtKB:Q96DM1"
}